{
  "gene": "UniProtKB:P07766",
  "term_id": "GO:0045059",
  "gene_symbol": "CD3E",
  "gene_name": "T-cell surface glycoprotein CD3 epsilon chain",
  "term_label": "positive thymic T cell selection"
}